{
  "gene": "UniProtKB:Q9UFV1",
  "gene_name": "Putative TBC1 domain family member 29",
  "gene_symbol": "TBC1D29P",
  "term_id": "UNKNOWN:0001",
  "term_label": "Unknown molecular function"
}